{
  "term_label": "Unknown cellular component",
  "gene_name": "Olfactory receptor 11H1",
  "term_id": "UNKNOWN:0003",
  "gene_symbol": "OR11H1",
  "gene": "UniProtKB:Q8NG94"
}